{
  "gene_symbol": "PLCD4",
  "gene": "UniProtKB:Q9BRC7",
  "gene_name": "1-phosphatidylinositol 4,5-bisphosphate phosphodiesterase delta-4",
  "term_label": "Unknown biological process",
  "term_id": "UNKNOWN:0002"
}